{
  "term_label": "microtubule motor activity",
  "gene_symbol": "KIF12",
  "term_id": "GO:0003777",
  "gene": "UniProtKB:Q96FN5",
  "gene_name": "Kinesin-like protein KIF12"
}